{
  "term_id": "UNKNOWN:0003",
  "gene": "UniProtKB:Q5T6L9",
  "gene_name": "Endoplasmic reticulum membrane-associated RNA degradation protein",
  "gene_symbol": "ERMARD",
  "term_label": "Unknown cellular component"
}